tumor necrosis factor receptor activity [GO:0005031] (molecular function) Sources: GOC:jl, http://lookwayup.com/ Definition: Combining with tumor necrosis factor, a proinflammatory cytokine produced by monocytes and macrophages, to initiate a change in cell function. Relationships: is a type of GO:0005035; is part of GO:0033209; has part tumor necrosis factor binding [GO:0043120] Also known as: TNF receptor activity, tumor necrosis factor-activated receptor activity, NGF/TNF (6 C-domain) receptor activity, TNF receptor activity, type I, TNF receptor activity, type II, tumor necrosis factor receptor activity, type I, tumor necrosis factor receptor activity, type II